light-harvesting complex, peripheral complex [GO:0030079] (cellular component) Definition: Bacteriochlorophyll a binding complex that is peripherally associated to the bacterial reaction center. Sources: GOC:lr Relationships: is a type of plasma membrane light-harvesting complex [GO:0030077]